negative regulation of developmental vegetative growth [GO:1905614] (biological process) Relationships: is_a negative regulation of developmental growth [GO:0048640]; is a type of regulation of developmental vegetative growth [GO:1905613]; negatively regulates developmental vegetative growth [GO:0080186] Also known as: down regulation of developmental vegetative growth, down-regulation of developmental vegetative growth, downregulation of developmental vegetative growth, inhibition of developmental vegetative growth Definition: Any process that stops, prevents or reduces the frequency, rate or extent of developmental vegetative growth. References: PMID:11606552 Sources: GOC:TermGenie, GO_REF:0000058